late meiotic recombination nodule assembly [GO:0042140] (biological process) Relationships: is a type of meiotic recombination nodule assembly [GO:0007146] Definition: During meiosis, the aggregation, arrangement and bonding together of strand exchange proteins (recombinases) to form small, electron dense structures in association with meiotic chromosomes during pachytene. Involved in the catalysis crossing over. References: PMID:9334324 Sources: GOC:jl